{
  "term_label": "regulation of transcription by RNA polymerase II",
  "gene": "UniProtKB:Q8IZ20",
  "gene_symbol": "ZNF683",
  "gene_name": "Tissue-resident T-cell transcription regulator protein ZNF683",
  "term_id": "GO:0006357"
}